{
  "term_label": "proteasome complex",
  "term_id": "GO:0000502",
  "gene": "UniProtKB:Q9BRP4",
  "gene_name": "Proteasomal ATPase-associated factor 1",
  "gene_symbol": "PAAF1"
}